imaginal disc-derived wing expansion [GO:0048526] (biological process) Definition: The process of expanding or inflating the folded imaginal disc-derived pupal wing, and the adhering of the dorsal and ventral surfaces, to form the mature adult wing. Relationships: is_a GO:0060560; BFO_0000050 GO:0007476 Sources: GOC:mtg_sensu, GOC:rc Also known as: wing expansion, wing inflation